{
  "term_label": "anatomical structure morphogenesis",
  "gene_name": "Mothers against decapentaplegic homolog 6",
  "gene_symbol": "SMAD6",
  "term_id": "GO:0009653",
  "gene": "UniProtKB:O43541"
}